{
  "term_id": "UNKNOWN:0001",
  "term_label": "Unknown molecular function",
  "gene": "UniProtKB:P20023",
  "gene_symbol": "CR2",
  "gene_name": "Complement receptor type 2"
}